cellular component disassembly [GO:0022411] (biological process) Sources: GOC:isa_complete Definition: A cellular process that results in the breakdown of a cellular component. Relationships: is a type of cellular component organization [GO:0016043] Subtypes: cellular component disassembly involved in execution phase of apoptosis [GO:0006921], extracellular matrix disassembly [GO:0022617], GO:0030397, GO:0030994, equatorial microtubule organizing center disassembly [GO:0031025], pseudopodium retraction [GO:0031270], protein-containing complex disassembly [GO:0032984], cell wall disassembly [GO:0044277], synaptonemal complex disassembly [GO:0070194], enucleation [GO:0090601], GO:0150146, organelle disassembly [GO:1903008], presynaptic active zone disassembly [GO:1904072], manchette disassembly [GO:1905199] Note: Note that this term is in the subset of terms that should not be used for direct gene product annotation. Instead, select a child term or, if no appropriate child term exists, please request a new term. Direct annotations to this term may be amended during annotation QC. Also known as: cell structure disassembly, cellular component disassembly at cellular level